{
  "gene_symbol": "ATXN7",
  "term_id": "UNKNOWN:0003",
  "gene_name": "Ataxin-7",
  "term_label": "Unknown cellular component",
  "gene": "UniProtKB:O15265"
}